{
  "gene_name": "CAAX box protein 1",
  "gene": "UniProtKB:O15255",
  "gene_symbol": "RTL8C",
  "term_label": "Unknown cellular component",
  "term_id": "UNKNOWN:0003"
}